{
  "gene_symbol": "KIT",
  "term_label": "cell migration",
  "gene": "UniProtKB:P10721",
  "term_id": "GO:0016477",
  "gene_name": "Mast_stem cell growth factor receptor Kit"
}